cardiac muscle thin filament assembly [GO:0071691] (biological process) Relationships: is a type of actin filament organization [GO:0007015]; is part of cardiac myofibril assembly [GO:0055003] Sources: GOC:mah Definition: The aggregation, arrangement and bonding together of proteins to form the actin-based thin filaments of myofibrils in cardiac muscle.